positive regulation of interleukin-27-mediated signaling pathway [GO:0070109] (biological process) Relationships: is a type of positive regulation of cytokine-mediated signaling pathway [GO:0001961]; is a type of GO:0070107; positively regulates interleukin-27-mediated signaling pathway [GO:0070106] Also known as: positive regulation of IL-27-mediated signaling pathway, positive regulation of IL27RA/IL6ST signaling pathway, positive regulation of interleukin-27-mediated signalling pathway Definition: Any process that increases the rate, frequency or extent of an interleukin-27-mediated signaling pathway. Sources: GOC:BHF, GOC:mah